{
  "gene_name": "Phosphoglycerate mutase 1",
  "term_label": "canonical glycolysis",
  "gene_symbol": "PGAM1",
  "term_id": "GO:0061621",
  "gene": "UniProtKB:P18669"
}